{
  "gene_name": "Zinc finger SWIM domain-containing protein 4",
  "gene": "UniProtKB:Q9H7M6",
  "term_label": "Unknown molecular function",
  "gene_symbol": "ZSWIM4",
  "term_id": "UNKNOWN:0001"
}